{
  "gene_name": "Multicilin",
  "term_label": "nucleus",
  "gene_symbol": "MCIDAS",
  "term_id": "GO:0005634",
  "gene": "UniProtKB:D6RGH6"
}